{
  "term_label": "actin filament binding",
  "gene": "UniProtKB:Q99501",
  "gene_symbol": "GAS2L1",
  "gene_name": "GAS2-like protein 1",
  "term_id": "GO:0051015"
}